{
  "gene_name": "TATA-box-binding protein-associated factor 11-like protein 4",
  "gene_symbol": "TAF11L4",
  "term_id": "GO:0016251",
  "term_label": "RNA polymerase II general transcription initiation factor activity",
  "gene": "UniProtKB:A0A1W2PPE2"
}